negative regulation of eosinophil migration [GO:2000417] (biological process) Subtypes: GO:2000420, GO:2000423 Sources: GOC:mah Relationships: is a type of negative regulation of leukocyte migration [GO:0002686]; is a type of regulation of eosinophil migration [GO:2000416]; negatively regulates GO:0072677 Definition: Any process that stops, prevents or reduces the frequency, rate or extent of eosinophil migration.